{
  "term_label": "immune response",
  "term_id": "GO:0006955",
  "gene_symbol": "TRAV2",
  "gene": "UniProtKB:A0A0B4J234",
  "gene_name": "T cell receptor alpha variable 2"
}